{
  "term_id": "GO:0008528",
  "gene_symbol": "LHCGR",
  "gene": "UniProtKB:P22888",
  "gene_name": "Lutropin-choriogonadotropic hormone receptor",
  "term_label": "G protein-coupled peptide receptor activity"
}